{
  "gene": "UniProtKB:P48382",
  "term_label": "RNA polymerase II cis-regulatory region sequence-specific DNA binding",
  "term_id": "GO:0000978",
  "gene_name": "DNA-binding protein RFX5",
  "gene_symbol": "RFX5"
}